{
  "gene": "UniProtKB:P63133",
  "term_id": "UNKNOWN:0002",
  "term_label": "Unknown biological process",
  "gene_name": "Endogenous retrovirus group K member 8 Pol protein",
  "gene_symbol": "ERVK-8"
}